{
  "gene_name": "Polypeptide N-acetylgalactosaminyltransferase 13",
  "term_id": "GO:0006493",
  "term_label": "protein O-linked glycosylation",
  "gene_symbol": "GALNT13",
  "gene": "UniProtKB:Q8IUC8"
}